{
  "term_id": "GO:0005783",
  "gene_symbol": "CLN8",
  "term_label": "endoplasmic reticulum",
  "gene": "UniProtKB:Q9UBY8",
  "gene_name": "Protein CLN8"
}